{
  "gene": "UniProtKB:O95163",
  "gene_symbol": "ELP1",
  "gene_name": "Elongator complex protein 1",
  "term_label": "tRNA binding",
  "term_id": "GO:0000049"
}